chromatin DNA binding [GO:0031490] (molecular function) Sources: GOC:mah Subtypes: nucleosomal DNA binding [GO:0031492], GO:0043035, chromatin loop anchoring activity [GO:0140587] Definition: Binding to DNA that is assembled into chromatin. Relationships: is a type of DNA binding [GO:0003677]; is a type of chromatin binding [GO:0003682]